regulation of reactive oxygen species metabolic process [GO:2000377] (biological process) Sources: GOC:mah Definition: Any process that modulates the frequency, rate or extent of reactive oxygen species metabolic process. Also known as: regulation of ROS metabolic process, regulation of reactive oxygen species metabolism Subtypes: regulation of hydrogen peroxide metabolic process [GO:0010310], GO:0090322, regulation of reactive oxygen species biosynthetic process [GO:1903426], GO:2000378, positive regulation of reactive oxygen species metabolic process [GO:2000379] Relationships: is a type of regulation of metabolic process [GO:0019222]; regulates reactive oxygen species metabolic process [GO:0072593]